{
  "gene_name": "Atrial natriuretic peptide receptor 2",
  "term_id": "GO:0005886",
  "gene": "UniProtKB:P20594",
  "term_label": "plasma membrane",
  "gene_symbol": "NPR2"
}